{
  "term_label": "Unknown cellular component",
  "gene_symbol": "RAVER1",
  "gene_name": "Ribonucleoprotein PTB-binding 1",
  "gene": "UniProtKB:Q8IY67",
  "term_id": "UNKNOWN:0003"
}